guanine transmembrane transporter activity [GO:0015208] (molecular function) Subtypes: ABC-type guanine transporter activity [GO:0008558] Sources: GOC:go_curators Definition: Enables the transfer of guanine, 2-amino-6-hydroxypurine, from one side of a membrane to the other. Relationships: is a type of GO:0005345; is part of guanine transmembrane transport [GO:1903716]